{
  "gene_symbol": "SEBOX",
  "term_label": "Unknown biological process",
  "gene_name": "Homeobox protein SEBOX",
  "gene": "UniProtKB:Q9HB31",
  "term_id": "UNKNOWN:0002"
}